{
  "gene_symbol": "RHCG",
  "gene": "UniProtKB:Q9UBD6",
  "gene_name": "Ammonium transporter Rh type C",
  "term_id": "GO:0016324",
  "term_label": "apical plasma membrane"
}